{
  "gene": "UniProtKB:Q7KZF4",
  "term_id": "GO:0005634",
  "term_label": "nucleus",
  "gene_name": "Staphylococcal nuclease domain-containing protein 1",
  "gene_symbol": "SND1"
}